post-embryonic plant organ development [GO:0090696] (biological process) Definition: Development, taking place during the post-embryonic phase of a plant tissue or tissues that work together to perform a specific function or functions. Development pertains to the process whose specific outcome is the progression of a structure over time, from its formation to the mature structure. Organs are commonly observed as visibly distinct structures, but may also exist as loosely associated clusters of cells that work together to perform a specific function or functions. Sources: GOC:tb Relationships: is a type of post-embryonic development [GO:0009791]; is a type of plant organ development [GO:0099402] Subtypes: GO:0048528